cellular response to cytokine stimulus [GO:0071345] (biological process) Definition: Any process that results in a change in state or activity of a cell (in terms of movement, secretion, enzyme production, gene expression, etc.) as a result of a cytokine stimulus. Sources: GOC:mah Relationships: is a type of response to cytokine [GO:0034097] Subtypes: cellular response to interferon-alpha [GO:0035457], cellular response to interferon-beta [GO:0035458], GO:0035963, cellular response to macrophage colony-stimulating factor stimulus [GO:0036006], GO:0036016, cellular response to erythropoietin [GO:0036018], cellular response to stem cell factor stimulus [GO:0036216], cellular response to type II interferon [GO:0071346], cellular response to interleukin-1 [GO:0071347], cellular response to interleukin-11 [GO:0071348], cellular response to interleukin-12 [GO:0071349], cellular response to interleukin-15 [GO:0071350], GO:0071351, GO:0071352, cellular response to interleukin-4 [GO:0071353], cellular response to interleukin-6 [GO:0071354], GO:0071355, cellular response to tumor necrosis factor [GO:0071356], cellular response to type I interferon [GO:0071357], GO:0071358, cellular response to granulocyte macrophage colony-stimulating factor stimulus [GO:0097011], cellular response to interleukin-32 [GO:0097397], cellular response to interleukin-17 [GO:0097398], GO:0098759, GO:0098761, GO:1990643, cellular response to leukemia inhibitory factor [GO:1990830], cellular response to chemokine [GO:1990869]